{
  "gene_name": "Putative WAS protein family homolog 3",
  "gene_symbol": "WASH3P",
  "term_label": "Arp2/3 complex-mediated actin nucleation",
  "term_id": "GO:0034314",
  "gene": "UniProtKB:C4AMC7"
}